{
  "term_label": "nucleus",
  "gene_name": "Cotranscriptional regulator FAM172A",
  "term_id": "GO:0005634",
  "gene_symbol": "ARB2A",
  "gene": "UniProtKB:Q8WUF8"
}